terpenoid metabolic process [GO:0006721] (biological process) Also known as: terpenoid metabolism Definition: The chemical reactions and pathways involving terpenoids, any member of a class of compounds characterized by an isoprenoid chemical structure and including derivatives with various functional groups. Sources: ISBN:0198506732 Relationships: is a type of GO:0006720 Subtypes: sesquiterpenoid metabolic process [GO:0006714], triterpenoid metabolic process [GO:0006722], monoterpenoid metabolic process [GO:0016098], diterpenoid metabolic process [GO:0016101], GO:0016114, terpenoid catabolic process [GO:0016115], carotenoid metabolic process [GO:0016116], geranyl diphosphate metabolic process [GO:0033383], geranylgeranyl diphosphate metabolic process [GO:0033385], GO:0045338